{
  "gene_name": "Bcl-2-like protein 15",
  "term_label": "Unknown molecular function",
  "term_id": "UNKNOWN:0001",
  "gene": "UniProtKB:Q5TBC7",
  "gene_symbol": "BCL2L15"
}